{
  "gene_name": "Arf-GAP with Rho-GAP domain, ANK repeat and PH domain-containing protein 1",
  "gene_symbol": "ARAP1",
  "term_label": "GTPase activator activity",
  "gene": "UniProtKB:Q96P48",
  "term_id": "GO:0005096"
}